pre-mRNA binding [GO:0036002] (molecular function) Also known as: protein-coding primary transcript binding Subtypes: pre-mRNA 5'-splice site binding [GO:0030627], GO:0030628, pre-mRNA branch point binding [GO:0045131], histone pre-mRNA stem-loop binding [GO:0071207], GO:0097157 Relationships: is_a RNA binding [GO:0003723] References: PMID:21901112 Sources: GOC:bf, GOC:kmv, SO:0000120 Definition: Binding to a pre-messenger RNA (pre-mRNA), an intermediate molecule between DNA and protein that may contain introns and, at least in part, encodes one or more proteins. Introns are removed from pre-mRNA to form a mRNA molecule.